{
  "gene_symbol": "N4BP2",
  "term_id": "UNKNOWN:0003",
  "gene": "UniProtKB:Q86UW6",
  "gene_name": "NEDD4-binding protein 2",
  "term_label": "Unknown cellular component"
}